negative regulation of leukocyte apoptotic process [GO:2000107] (biological process) Also known as: negative regulation of leukocyte apoptosis Definition: Any process that stops, prevents, or reduces the frequency, rate or extent of leukocyte apoptotic process. Sources: GOC:BHF, GOC:mtg_apoptosis Relationships: is a type of negative regulation of apoptotic process [GO:0043066]; is a type of regulation of leukocyte apoptotic process [GO:2000106]; negatively regulates leukocyte apoptotic process [GO:0071887] Subtypes: negative regulation of mast cell apoptotic process [GO:0033026], negative regulation of neutrophil apoptotic process [GO:0033030], negative regulation of lymphocyte apoptotic process [GO:0070229], GO:2000110, GO:2000669